{
  "gene": "UniProtKB:O14709",
  "gene_name": "Zinc finger protein 197",
  "term_id": "GO:0006357",
  "term_label": "regulation of transcription by RNA polymerase II",
  "gene_symbol": "ZNF197"
}